{
  "gene": "UniProtKB:Q9UGI6",
  "term_label": "neuron projection",
  "term_id": "GO:0043005",
  "gene_symbol": "KCNN3",
  "gene_name": "Small conductance calcium-activated potassium channel protein 3"
}